{
  "gene_symbol": "PCK1",
  "gene": "UniProtKB:P35558",
  "term_label": "oxaloacetate metabolic process",
  "gene_name": "Phosphoenolpyruvate carboxykinase, cytosolic [GTP]",
  "term_id": "GO:0006107"
}